{
  "gene_name": "Cytokine receptor-like factor 3",
  "gene": "UniProtKB:Q8IUI8",
  "gene_symbol": "CRLF3",
  "term_label": "Unknown biological process",
  "term_id": "UNKNOWN:0002"
}